negative regulation of muscle filament sliding [GO:1904113] (biological process) References: PMID:25717181 Sources: GOC:TermGenie, GOC:kmv, GO_REF:0000058 Also known as: down regulation of muscle filament sliding, down-regulation of muscle filament sliding, downregulation of muscle filament sliding, inhibition of muscle filament sliding Relationships: is a type of regulation of muscle filament sliding [GO:0032971]; is a type of GO:0045932; is a type of negative regulation of cellular process [GO:0048523]; negatively regulates muscle filament sliding [GO:0030049] Definition: Any process that stops, prevents or reduces the frequency, rate or extent of muscle filament sliding.